{
  "term_label": "melanosome",
  "gene_symbol": "MREG",
  "gene_name": "Melanoregulin",
  "gene": "UniProtKB:Q8N565",
  "term_id": "GO:0042470"
}